{
  "gene_name": "Sodium- and chloride-dependent neutral and basic amino acid transporter B(0+)",
  "term_id": "GO:0005886",
  "gene": "UniProtKB:Q9UN76",
  "gene_symbol": "SLC6A14",
  "term_label": "plasma membrane"
}